{
  "gene_symbol": "GLI1",
  "term_label": "nucleus",
  "gene": "UniProtKB:P08151",
  "gene_name": "Zinc finger protein GLI1",
  "term_id": "GO:0005634"
}